{
  "gene": "UniProtKB:Q96N68",
  "gene_symbol": "C18orf15",
  "term_label": "Unknown molecular function",
  "gene_name": "Putative uncharacterized protein C18orf15",
  "term_id": "UNKNOWN:0001"
}